{
  "term_label": "mitochondrion",
  "gene_symbol": "IVD",
  "gene": "UniProtKB:P26440",
  "gene_name": "Isovaleryl-CoA dehydrogenase, mitochondrial",
  "term_id": "GO:0005739"
}